{
  "gene": "UniProtKB:Q70CQ4",
  "gene_name": "Ubiquitin carboxyl-terminal hydrolase 31",
  "term_id": "UNKNOWN:0002",
  "gene_symbol": "USP31",
  "term_label": "Unknown biological process"
}